{
  "gene": "UniProtKB:P58182",
  "gene_name": "Olfactory receptor 12D2",
  "gene_symbol": "OR12D2",
  "term_label": "membrane",
  "term_id": "GO:0016020"
}